{
  "gene": "UniProtKB:Q9NSE4",
  "gene_symbol": "IARS2",
  "term_label": "isoleucyl-tRNA aminoacylation",
  "gene_name": "Isoleucine--tRNA ligase, mitochondrial",
  "term_id": "GO:0006428"
}